{
  "gene_name": "Autoimmune regulator",
  "term_id": "GO:0002458",
  "term_label": "peripheral T cell tolerance induction",
  "gene": "UniProtKB:O43918",
  "gene_symbol": "AIRE"
}